{
  "gene_name": "Lysosomal alpha-mannosidase",
  "term_label": "Unknown biological process",
  "term_id": "UNKNOWN:0002",
  "gene": "UniProtKB:O00754",
  "gene_symbol": "MAN2B1"
}